{
  "term_id": "UNKNOWN:0003",
  "term_label": "Unknown cellular component",
  "gene_symbol": "SERTAD4-AS1",
  "gene_name": "Putative uncharacterized protein SERTAD4-AS1",
  "gene": "UniProtKB:Q5TG53"
}